{
  "term_label": "Unknown cellular component",
  "gene": "UniProtKB:Q92583",
  "gene_name": "C-C motif chemokine 17",
  "gene_symbol": "CCL17",
  "term_id": "UNKNOWN:0003"
}